{
  "gene": "UniProtKB:P35367",
  "gene_symbol": "HRH1",
  "term_label": "G protein-coupled receptor signaling pathway, coupled to cyclic nucleotide second messenger",
  "term_id": "GO:0007187",
  "gene_name": "Histamine H1 receptor"
}